{
  "gene_symbol": "NCF1",
  "gene": "UniProtKB:P14598",
  "term_label": "NADPH oxidase complex",
  "gene_name": "Neutrophil cytosol factor 1",
  "term_id": "GO:0043020"
}